{
  "term_label": "nuclear membrane",
  "gene_symbol": "SYNE1",
  "gene_name": "Nesprin-1",
  "gene": "UniProtKB:Q8NF91",
  "term_id": "GO:0031965"
}